collagen fibril binding [GO:0098633] (molecular function) Relationships: is a type of extracellular matrix binding [GO:0050840] Definition: Binding to a collagen fibril. References: PMID:21421911 Sources: GOC:dos